U2 snRNA 3'-end processing [GO:0034474] (biological process) Sources: GOC:mah Definition: Any process involved in forming the mature 3' end of a U2 snRNA molecule. Also known as: U2 snRNA 3' end processing Relationships: is a type of GO:0034472